{
  "gene": "UniProtKB:Q96M27",
  "term_id": "GO:0010669",
  "term_label": "epithelial structure maintenance",
  "gene_symbol": "PRRC1",
  "gene_name": "Protein PRRC1"
}